{
  "gene_name": "Apolipoprotein A-II",
  "term_label": "spherical high-density lipoprotein particle",
  "gene_symbol": "APOA2",
  "gene": "UniProtKB:P02652",
  "term_id": "GO:0034366"
}